response to gastrin [GO:1990867] (biological process) Definition: Any process that results in a change in state or activity of a cell or an organism (in terms of movement, secretion, enzyme production, gene expression, etc.) as a result of a gastrin stimulus. References: PMID:10348814 Subtypes: cellular response to gastrin [GO:1990878] Relationships: is a type of GO:0043434